{
  "gene_symbol": "ZIC3",
  "gene_name": "Zinc finger protein ZIC 3",
  "term_id": "GO:0005634",
  "term_label": "nucleus",
  "gene": "UniProtKB:O60481"
}